{
  "term_id": "GO:0045087",
  "gene": "UniProtKB:Q99969",
  "term_label": "innate immune response",
  "gene_name": "Retinoic acid receptor responder protein 2",
  "gene_symbol": "RARRES2"
}